{
  "gene_name": "Mothers against decapentaplegic homolog 3",
  "gene_symbol": "SMAD3",
  "term_label": "anatomical structure morphogenesis",
  "gene": "UniProtKB:P84022",
  "term_id": "GO:0009653"
}